{
  "gene_name": "Leucine-rich repeat-containing protein 74A",
  "term_id": "UNKNOWN:0001",
  "term_label": "Unknown molecular function",
  "gene": "UniProtKB:Q0VAA2",
  "gene_symbol": "LRRC74A"
}